{
  "gene": "UniProtKB:Q8N371",
  "term_id": "GO:0106157",
  "gene_symbol": "KDM8",
  "term_label": "peptidyl-arginine 3-dioxygenase activity",
  "gene_name": "Bifunctional peptidase and arginyl-hydroxylase JMJD5"
}